{
  "gene": "UniProtKB:P23975",
  "gene_symbol": "SLC6A2",
  "term_label": "plasma membrane",
  "gene_name": "Sodium-dependent noradrenaline transporter",
  "term_id": "GO:0005886"
}